{
  "term_id": "GO:0016020",
  "gene_symbol": "MYO5A",
  "term_label": "membrane",
  "gene_name": "Unconventional myosin-Va",
  "gene": "UniProtKB:Q9Y4I1"
}